{
  "gene": "UniProtKB:O75185",
  "gene_symbol": "ATP2C2",
  "term_id": "GO:0005388",
  "term_label": "P-type calcium transporter activity",
  "gene_name": "Calcium-transporting ATPase type 2C member 2"
}